{
  "gene_name": "ATP-dependent RNA helicase DDX3Y",
  "gene_symbol": "DDX3Y",
  "term_id": "GO:0030154",
  "gene": "UniProtKB:O15523",
  "term_label": "cell differentiation"
}